{
  "gene_name": "High affinity cAMP-specific and IBMX-insensitive 3',5'-cyclic phosphodiesterase 8B",
  "term_label": "3',5'-cyclic-GMP phosphodiesterase activity",
  "gene_symbol": "PDE8B",
  "term_id": "GO:0047555",
  "gene": "UniProtKB:O95263"
}